{
  "gene_symbol": "ETFA",
  "term_label": "fatty acid beta-oxidation using acyl-CoA dehydrogenase",
  "gene": "UniProtKB:P13804",
  "term_id": "GO:0033539",
  "gene_name": "Electron transfer flavoprotein subunit alpha, mitochondrial"
}